{
  "gene_symbol": "CSNK2A3",
  "term_id": "GO:0005634",
  "gene": "UniProtKB:Q8NEV1",
  "term_label": "nucleus",
  "gene_name": "Casein kinase II subunit alpha 3"
}